{
  "gene": "UniProtKB:Q9BY78",
  "term_label": "ubiquitin-dependent protein catabolic process",
  "term_id": "GO:0006511",
  "gene_name": "E3 ubiquitin-protein ligase RNF26",
  "gene_symbol": "RNF26"
}